{
  "term_id": "GO:0005886",
  "gene": "UniProtKB:A6NI73",
  "gene_symbol": "LILRA5",
  "gene_name": "Leukocyte immunoglobulin-like receptor subfamily A member 5",
  "term_label": "plasma membrane"
}